{
  "gene_symbol": "SLC2A11",
  "term_label": "plasma membrane",
  "gene_name": "Solute carrier family 2, facilitated glucose transporter member 11",
  "term_id": "GO:0005886",
  "gene": "UniProtKB:Q9BYW1"
}